{
  "gene": "UniProtKB:Q9NRH2",
  "term_id": "GO:0004674",
  "term_label": "protein serine/threonine kinase activity",
  "gene_symbol": "SNRK",
  "gene_name": "SNF-related serine_threonine-protein kinase"
}